{
  "gene_symbol": "ATG4B",
  "term_id": "GO:0000045",
  "gene_name": "Cysteine protease ATG4B",
  "gene": "UniProtKB:Q9Y4P1",
  "term_label": "autophagosome assembly"
}